viral RNA genome packaging [GO:0019074] (BP) Relationships: is a type of GO:0019072 Sources: ISBN:0781718325 Definition: The packaging of viral RNA (single-stranded or double-stranded) into a nucleocapsid.